T cell apoptotic process [GO:0070231] (biological process) Definition: Any apoptotic process in a T cell, a type of lymphocyte whose defining characteristic is the expression of a T cell receptor complex. Sources: CL:0000084, GOC:add, GOC:mtg_apoptosis, ISBN:0781765196 Also known as: T lymphocyte apoptosis, T-cell apoptosis, T-lymphocyte apoptosis, programmed cell death of T cells by apoptosis, T cell apoptosis Relationships: is_a lymphocyte apoptotic process [GO:0070227] Subtypes: activation-induced cell death of T cells [GO:0006924], GO:0070238, thymocyte apoptotic process [GO:0070242], regulatory T cell apoptotic process [GO:1902482], activated CD8-positive, alpha-beta T cell apoptotic process [GO:1905397], activated CD4-positive, alpha-beta T cell apoptotic process [GO:1905398] Regulation: regulated by regulation of T cell apoptotic process [GO:0070232]; negatively regulated by negative regulation of T cell apoptotic process [GO:0070233]; positively regulated by positive regulation of T cell apoptotic process [GO:0070234]